Maurer's cleft [GO:0020036] (cellular component) Also known as: Maurers cleft Definition: A disk-like structure that appears at the periphery of a red blood cell infected by an apicomplexan parasite, characterized by a translucent lumen and an electron-dense coat of variable thickness; often appears to be tethered to the host cell membrane by fibrous connections with the erythrocyte cytoskeleton. Relationships: is a type of GO:0033655 References: PMID:16705161